lung-associated mesenchyme development [GO:0060484] (biological process) Relationships: is a type of mesenchyme development [GO:0060485]; is part of lung development [GO:0030324] Sources: GOC:dph, GOC:mtg_lung Subtypes: GO:0060483 Also known as: lung mesenchyme development, pulmonary mesenchyme development Definition: The biological process whose specific outcome is the progression of a lung-associated mesenchyme from an initial condition to its mature state. This process begins with the formation of lung-associated mesenchyme and ends with the mature structure. Lung-associated mesenchyme is the tissue made up of loosely connected mesenchymal cells in the lung.